{
  "term_label": "cell fate specification",
  "gene_name": "T-box transcription factor TBX18",
  "gene_symbol": "TBX18",
  "gene": "UniProtKB:O95935",
  "term_id": "GO:0001708"
}